{
  "gene_symbol": "H2BC5",
  "term_id": "GO:0030527",
  "term_label": "structural constituent of chromatin",
  "gene_name": "Histone H2B type 1-D",
  "gene": "UniProtKB:P58876"
}